P3 peroxisome [GO:0019821] (cellular component) Note: Note that this peroxisome assembly pathway is described in the yeast Yarrowia lipolytica. See also the cellular component terms 'P1 peroxisome ; GO:0019819', 'P2 peroxisome ; GO:0019820', 'P4 peroxisome ; GO:0019822', 'P5 peroxisome ; GO:0019823', and 'P6 peroxisome ; GO:0019824'. Relationships: is a type of peroxisome [GO:0005777] References: PMID:10629216 Also known as: peroxisome vesicle Definition: A subform of peroxisome that corresponds to an intermediate in a peroxisome assembly pathway, which operates by conversion of peroxisomal subforms in the direction P1, P2 -> P3 -> P4 -> P5 -> P6. P3 peroxisomes are formed by fusion of P1 and P2 peroxisomes, and are distinguished from the other subforms on the bases of buoyant density and protein content.